isoprenoid biosynthetic process via 1-deoxy-D-xylulose 5-phosphate [GO:1902768] (biological process) Definition: The chemical reactions and pathways resulting in the formation of isoprenoid via 1-deoxy-D-xylulose 5-phosphate. Also known as: isoprenoid anabolism via 1-deoxy-D-xylulose 5-phosphate, isoprenoid biosynthesis via 1-deoxy-D-xylulose 5-phosphate, isoprenoid formation via 1-deoxy-D-xylulose 5-phosphate, isoprenoid synthesis via 1-deoxy-D-xylulose 5-phosphate References: PMID:23746261 Sources: GOC:TermGenie, GOC:mengo_curators, GO_REF:0000092 Relationships: is a type of isoprenoid biosynthetic process [GO:0008299]